negative regulation of glucuronoarabinoxylan catabolic process [GO:2000919] (biological process) Definition: Any process that stops, prevents or reduces the frequency, rate or extent of glucuronoarabinoxylan catabolic process. Sources: GOC:mengo_curators Also known as: negative regulation of glucuronoarabinoxylan catabolism Relationships: is a type of negative regulation of glucuronoxylan catabolic process [GO:2000916]; is a type of regulation of glucuronoarabinoxylan catabolic process [GO:2000918]; is a type of negative regulation of arabinoxylan-containing compound catabolic process [GO:2000922]; negatively regulates glucuronoarabinoxylan catabolic process [GO:2000887]